{
  "gene_symbol": "ZBTB40",
  "term_id": "GO:0000981",
  "gene": "UniProtKB:Q9NUA8",
  "term_label": "DNA-binding transcription factor activity, RNA polymerase II-specific",
  "gene_name": "Zinc finger and BTB domain-containing protein 40"
}